metanephric mesangial cell differentiation [GO:0072209] (biological process) Sources: GOC:mtg_kidney_jan10 Definition: The process in which relatively unspecialized cells acquire specialized structural and/or functional features that characterize the mesangial cells of the metanephros as it progresses from its formation to the mature state. Subtypes: metanephric glomerular mesangial cell differentiation [GO:0072254] Relationships: is a type of GO:0072007; is_a cell differentiation involved in metanephros development [GO:0072202]